{
  "gene_symbol": "FAM210B",
  "term_label": "mitochondrion",
  "gene": "UniProtKB:Q96KR6",
  "gene_name": "Protein FAM210B, mitochondrial",
  "term_id": "GO:0005739"
}